cis-abienol catabolic process [GO:1902245] (biological process) References: PMID:22672125 Sources: GOC:TermGenie Also known as: cis-abienol breakdown, cis-abienol catabolism, cis-abienol degradation Definition: The chemical reactions and pathways resulting in the breakdown of cis-abienol. Relationships: is a type of diterpenoid catabolic process [GO:0016103]; is a type of alcohol catabolic process [GO:0046164]; is a type of tertiary alcohol metabolic process [GO:1902644]